{
  "gene_name": "Bcl-2-like protein 1",
  "term_id": "GO:0005741",
  "term_label": "mitochondrial outer membrane",
  "gene_symbol": "BCL2L1",
  "gene": "UniProtKB:Q07817"
}